{
  "gene": "UniProtKB:Q9BYI3",
  "term_label": "Unknown molecular function",
  "term_id": "UNKNOWN:0001",
  "gene_name": "Hyccin",
  "gene_symbol": "HYCC1"
}